{
  "gene": "UniProtKB:Q9NQ75",
  "term_id": "UNKNOWN:0001",
  "gene_name": "Cas scaffolding protein family member 4",
  "gene_symbol": "CASS4",
  "term_label": "Unknown molecular function"
}